{
  "gene_name": "ETS translocation variant 4",
  "term_id": "GO:0005634",
  "gene_symbol": "ETV4",
  "term_label": "nucleus",
  "gene": "UniProtKB:P43268"
}